{
  "gene_symbol": "NEO1",
  "gene": "UniProtKB:Q92859",
  "term_id": "GO:0007411",
  "term_label": "axon guidance",
  "gene_name": "Neogenin"
}